female germ-line cyst encapsulation [GO:0048139] (biological process) Relationships: is a type of GO:0048138; is part of female gamete generation [GO:0007292] Subtypes: germarium-derived female germ-line cyst encapsulation [GO:0030708] Sources: GOC:jid Definition: Formation of a single follicular epithelium around the germ-line derived cells of a cyst formed in the female gonad.